positive regulation of thyroid-stimulating hormone secretion [GO:2000614] (biological process) Definition: Any process that activates or increases the frequency, rate or extent of thyroid-stimulating hormone secretion. Also known as: positive regulation of TSH secretion, positive regulation of thyroid stimulating hormone secretion Sources: GOC:obol Relationships: is a type of positive regulation of peptide hormone secretion [GO:0090277]; is a type of GO:2000612; positively regulates thyroid-stimulating hormone secretion [GO:0070460]